{
  "term_id": "GO:0045095",
  "term_label": "keratin filament",
  "gene_symbol": "KRT78",
  "gene": "UniProtKB:Q8N1N4",
  "gene_name": "Keratin, type II cytoskeletal 78"
}